cytochrome o ubiquinol oxidase complex [GO:0009319] (cellular component) Note: See also the molecular function term 'cytochrome o ubiquinol oxidase activity ; GO:0008827'. References: PMID:11017202, PMID:3052268 Sources: GOC:mah, MetaCyc:CYT-O-UBIOX-CPLX Relationships: is a type of cytochrome complex [GO:0070069]; is_a respiratory chain complex [GO:0098803]; is a type of transmembrane transporter complex [GO:1902495]; is a type of oxidoreductase complex [GO:1990204] Definition: A protein complex that possesses cytochrome o ubiquinol oxidase activity; consists of four polypeptide subunits and associated prosthetic groups.